{
  "gene_symbol": "H2BC1",
  "gene": "UniProtKB:Q96A08",
  "gene_name": "Histone H2B type 1-A",
  "term_id": "GO:0000786",
  "term_label": "nucleosome"
}